{
  "gene_name": "Alpha-soluble NSF attachment protein",
  "term_label": "regulation of synaptic vesicle priming",
  "gene": "UniProtKB:P54920",
  "gene_symbol": "NAPA",
  "term_id": "GO:0010807"
}